{
  "gene": "UniProtKB:Q92928",
  "gene_symbol": "RAB1C",
  "term_label": "intracellular protein transport",
  "gene_name": "Putative Ras-related protein Rab-1C",
  "term_id": "GO:0006886"
}